{
  "term_label": "regulation of DNA-templated transcription",
  "term_id": "GO:0006355",
  "gene_name": "High mobility group protein HMG-I_HMG-Y",
  "gene_symbol": "HMGA1",
  "gene": "UniProtKB:P17096"
}